{
  "gene_symbol": "PPP1R27",
  "gene_name": "Protein phosphatase 1 regulatory subunit 27",
  "term_label": "Unknown cellular component",
  "term_id": "UNKNOWN:0003",
  "gene": "UniProtKB:Q86WC6"
}